{
  "gene_symbol": "PRR25",
  "gene_name": "Proline-rich protein 25",
  "term_id": "UNKNOWN:0002",
  "gene": "UniProtKB:Q96S07",
  "term_label": "Unknown biological process"
}